{
  "term_id": "GO:0000981",
  "gene": "UniProtKB:Q9UPW6",
  "term_label": "DNA-binding transcription factor activity, RNA polymerase II-specific",
  "gene_symbol": "SATB2",
  "gene_name": "DNA-binding protein SATB2"
}